{
  "term_label": "negative regulation of apoptotic process",
  "gene": "UniProtKB:Q13490",
  "gene_symbol": "BIRC2",
  "term_id": "GO:0043066",
  "gene_name": "Baculoviral IAP repeat-containing protein 2"
}